BLOC-3 complex [GO:0031085] (cellular component) Relationships: is_a BLOC complex [GO:0031082] References: PMID:12756248 Definition: A protein complex required for the biogenesis of specialized organelles of the endosomal-lysosomal system, such as melanosomes and platelet dense granules. The human complex contains the Hps1 and Hps4 proteins.